{
  "gene": "UniProtKB:P52888",
  "term_id": "UNKNOWN:0002",
  "gene_symbol": "THOP1",
  "gene_name": "Thimet oligopeptidase",
  "term_label": "Unknown biological process"
}